mast cell migration [GO:0097531] (biological process) References: PMID:24152847 Sources: GOC:cvs Subtypes: mast cell chemotaxis [GO:0002551] Definition: The movement of a mast cell within or between different tissues and organs of the body. Relationships: is a type of GO:0097529